inner layer of spore wall [GO:0005632] (cellular component) Definition: Either of the two innermost layers of the spore wall, as described in Saccharomyces. Sources: ISBN:0879693568 Relationships: is a type of cellular anatomical structure [GO:0110165]; is part of GO:0005619